{
  "gene_symbol": "PLCZ1",
  "gene": "UniProtKB:Q86YW0",
  "term_label": "positive regulation of cytosolic calcium ion concentration involved in egg activation",
  "term_id": "GO:0060470",
  "gene_name": "1-phosphatidylinositol 4,5-bisphosphate phosphodiesterase zeta-1"
}